{
  "term_id": "GO:0005737",
  "gene": "UniProtKB:Q8WWB5",
  "term_label": "cytoplasm",
  "gene_name": "PIH1 domain-containing protein 2",
  "gene_symbol": "PIH1D2"
}